{
  "gene": "UniProtKB:Q96CM4",
  "term_id": "GO:0005739",
  "gene_name": "Nucleoredoxin-like protein 1",
  "gene_symbol": "NXNL1",
  "term_label": "mitochondrion"
}